{
  "gene": "UniProtKB:P00813",
  "term_label": "regulation of circadian sleep/wake cycle, sleep",
  "gene_symbol": "ADA",
  "term_id": "GO:0045187",
  "gene_name": "Adenosine deaminase"
}